protein tyrosine kinase activator activity [GO:0030296] (molecular function) Relationships: is a type of protein kinase activator activity [GO:0030295]; RO_0002213 protein tyrosine kinase activity [GO:0004713] Subtypes: transmembrane receptor protein tyrosine kinase activator activity [GO:0030297], GO:0030298 Sources: GOC:ai, ISBN:0198506732 Definition: Increases the activity of a protein tyrosine kinase, an enzyme which phosphorylates a tyrosyl phenolic group on a protein.